sorocarp stalk development [GO:0031150] (biological process) Definition: The process whose specific outcome is the progression of the sorocarp stalk over time, from its formation to the mature structure. The sorocarp stalk is a tubular structure that consists of cellulose-covered cells stacked on top of each other and surrounded by an acellular stalk tube composed of cellulose and glycoprotein. An example of this process is found in Dictyostelium discoideum. Relationships: is a type of socially cooperative development [GO:0099120]; is part of culmination involved in sorocarp development [GO:0031154] Also known as: stalk development, stalk formation, sorophore development References: PMID:4338436 Sources: GOC:mtg_sensu, ISBN:0521583640